{
  "gene": "UniProtKB:O95425",
  "gene_symbol": "SVIL",
  "gene_name": "Supervillin",
  "term_id": "GO:0008154",
  "term_label": "actin polymerization or depolymerization"
}